negative regulation of oogonium development [GO:0075266] (biological process) Definition: Any process that stops, prevents, or reduces the frequency, rate or extent of oogonium development, a process that leads to the formation of a female gametangium of oomycetes, containing one or more gametes. Sources: GOC:pamgo_curators Relationships: is a type of negative regulation of spore-bearing organ development [GO:0075262]; is_a regulation of oogonium development [GO:0075264]; negatively regulates oogonium development [GO:0075263]